chloromuconate cycloisomerase activity [GO:0018850] (molecular function) Relationships: is a type of intramolecular lyase activity [GO:0016872] Sources: EC:5.5.1.7 Also known as: 2-chloro-2,5-dihydro-5-oxofuran-2-acetate lyase (decyclizing), muconate cycloisomerase II activity Definition: Catalysis of the reaction: 2-chloro-2,5-dihydro-5-oxofuran-2-acetate = 3-chloro-cis,cis-muconate.